positive regulation of tetrapyrrole catabolic process [GO:1901406] (BP) Definition: Any process that activates or increases the frequency, rate or extent of tetrapyrrole catabolic process. Sources: GOC:TermGenie, GOC:mengo_curators Also known as: activation of tetrapyrrole breakdown, activation of tetrapyrrole catabolism, activation of tetrapyrrole degradation, positive regulation of tetrapyrrole breakdown, positive regulation of tetrapyrrole catabolism, positive regulation of tetrapyrrole degradation, up regulation of tetrapyrrole breakdown, up regulation of tetrapyrrole catabolic process, up regulation of tetrapyrrole catabolism, up regulation of tetrapyrrole degradation, up-regulation of tetrapyrrole breakdown, up-regulation of tetrapyrrole catabolic process, up-regulation of tetrapyrrole catabolism, up-regulation of tetrapyrrole degradation, upregulation of tetrapyrrole breakdown, upregulation of tetrapyrrole catabolic process, upregulation of tetrapyrrole catabolism, upregulation of tetrapyrrole degradation, activation of tetrapyrrole catabolic process Relationships: is a type of positive regulation of catabolic process [GO:0009896]; is a type of regulation of tetrapyrrole catabolic process [GO:1901404]; positively regulates tetrapyrrole catabolic process [GO:0033015] Subtypes: positive regulation of chlorophyll catabolic process [GO:1903648]